{
  "gene_symbol": "XCL1",
  "term_label": "positive regulation of cell migration",
  "gene_name": "Lymphotactin",
  "term_id": "GO:0030335",
  "gene": "UniProtKB:P47992"
}